protoderm histogenesis [GO:0010068] (biological process) Definition: The formation of the primary meristem or meristematic tissue that gives rise to the epidermis. Sources: GOC:tb, ISBN:0471245208 Relationships: is a type of primary meristem tissue development [GO:0010065]